{
  "term_label": "Unknown molecular function",
  "gene_name": "G antigen 12B_C_D_E",
  "gene": "UniProtKB:A1L429",
  "gene_symbol": "GAGE12E",
  "term_id": "UNKNOWN:0001"
}